{
  "gene_name": "Transmembrane and death domain protein 1",
  "term_label": "Unknown biological process",
  "gene_symbol": "TMDD1",
  "gene": "UniProtKB:P0DPE3",
  "term_id": "UNKNOWN:0002"
}